{
  "term_id": "GO:0005739",
  "gene_name": "Diablo IAP-binding mitochondrial protein",
  "gene_symbol": "DIABLO",
  "gene": "UniProtKB:Q9NR28",
  "term_label": "mitochondrion"
}